{
  "term_id": "GO:0016020",
  "gene": "UniProtKB:Q99685",
  "term_label": "membrane",
  "gene_symbol": "MGLL",
  "gene_name": "Monoglyceride lipase"
}